{
  "term_label": "G protein-coupled receptor signaling pathway",
  "gene_symbol": "GNG10",
  "term_id": "GO:0007186",
  "gene_name": "Guanine nucleotide-binding protein G(I)_G(S)_G(O) subunit gamma-10",
  "gene": "UniProtKB:P50151"
}